{
  "gene_name": "Peroxisome biogenesis factor 2",
  "gene_symbol": "PEX2",
  "term_label": "Unknown molecular function",
  "term_id": "UNKNOWN:0001",
  "gene": "UniProtKB:P28328"
}